{
  "gene_symbol": "POLDIP2",
  "gene": "UniProtKB:Q9Y2S7",
  "gene_name": "Polymerase delta-interacting protein 2",
  "term_label": "nucleus",
  "term_id": "GO:0005634"
}